{
  "gene_symbol": "C5orf60",
  "gene_name": "Uncharacterized protein C5orf60",
  "gene": "UniProtKB:A6NFR6",
  "term_label": "Unknown biological process",
  "term_id": "UNKNOWN:0002"
}